recurrent axon collateral [GO:1990020] (cellular component) Sources: NIF_Subcellular:sao1642494436 Definition: Axon collateral that ramifies in the area of the soma of the cell of origin. Relationships: is a type of axon collateral [GO:0044303] Also known as: recurrent collateral